{
  "gene_name": "Ankyrin repeat domain-containing protein 55",
  "term_id": "UNKNOWN:0003",
  "gene": "UniProtKB:Q3KP44",
  "gene_symbol": "ANKRD55",
  "term_label": "Unknown cellular component"
}